sucrose transport [GO:0015770] (biological process) Subtypes: phloem sucrose loading [GO:0009915], phloem sucrose unloading [GO:0110128], sucrose transmembrane transport [GO:1904982] Definition: The directed movement of sucrose into, out of or within a cell, or between cells by means of some agent such as a transporter or pore. Sucrose is the disaccharide fructofuranosyl-glucopyranoside. Relationships: is a type of disaccharide transport [GO:0015766] Sources: GOC:ai